{
  "term_id": "UNKNOWN:0002",
  "gene_symbol": "HIDE1",
  "gene_name": "Protein HIDE1",
  "gene": "UniProtKB:A8MVS5",
  "term_label": "Unknown biological process"
}